{
  "term_id": "GO:0005634",
  "gene": "UniProtKB:Q14995",
  "term_label": "nucleus",
  "gene_symbol": "NR1D2",
  "gene_name": "Nuclear receptor subfamily 1 group D member 2"
}